{
  "gene_name": "Protein FAM91A1",
  "term_id": "GO:0006886",
  "gene_symbol": "FAM91A1",
  "term_label": "intracellular protein transport",
  "gene": "UniProtKB:Q658Y4"
}